metanephric distal tubule morphogenesis [GO:0072287] (biological process) Relationships: is a type of distal tubule morphogenesis [GO:0072156]; is_a metanephric nephron tubule morphogenesis [GO:0072282]; is part of metanephric distal tubule development [GO:0072235] Definition: The process in which the anatomical structures of a metanephric distal tubule are generated and organized. The metanephric distal tubule is a metanephric nephron tubule that begins at the macula densa and extends to the metanephric connecting tubule. Sources: GOC:mtg_kidney_jan10